{
  "gene_symbol": "RMDN1",
  "term_id": "GO:0005739",
  "gene": "UniProtKB:Q96DB5",
  "term_label": "mitochondrion",
  "gene_name": "Regulator of microtubule dynamics protein 1"
}